{
  "gene_symbol": "REELD1",
  "term_id": "UNKNOWN:0001",
  "gene_name": "Reelin domain-containing protein 1",
  "gene": "UniProtKB:A0A1B0GV85",
  "term_label": "Unknown molecular function"
}